{
  "gene_name": "Protein phosphatase Slingshot homolog 3",
  "gene": "UniProtKB:Q8TE77",
  "term_label": "negative regulation of actin filament polymerization",
  "gene_symbol": "SSH3",
  "term_id": "GO:0030837"
}